eugenol catabolic process [GO:0042856] (biological process) Also known as: 4-allyl-2-methoxyphenol catabolic process, 4-allyl-2-methoxyphenol catabolism, eugenic acid catabolic process, eugenic acid catabolism, eugenol breakdown, eugenol catabolism, eugenol degradation Relationships: is a type of phenol-containing compound catabolic process [GO:0019336]; is_a eugenol metabolic process [GO:0042854]; is a type of phenylpropanoid catabolic process [GO:0046271]; is a type of olefinic compound catabolic process [GO:0120256]; is a type of ether catabolic process [GO:1901502] Sources: GOC:jl Definition: The chemical reactions and pathways resulting in the breakdown of eugenol, a colorless, aromatic, liquid hydrocarbon (C10H12O2) found in clove oil.